peptidyl-L-3-phenyllactic acid biosynthetic process from peptidyl-phenylalanine [GO:0018061] (biological process) Also known as: peptidyl-L-3-phenyllactic acid anabolism from peptidyl-phenylalanine, peptidyl-L-3-phenyllactic acid formation from peptidyl-phenylalanine, peptidyl-L-3-phenyllactic acid synthesis from peptidyl-phenylalanine Relationships: is a type of GO:0018207 Definition: The modification of a N-terminal peptidyl-phenylalanine residue by either oxidative deamination or by transamination and subsequent reduction to form peptidyl-L-3-phenyllactic acid. Sources: RESID:AA0128